{
  "gene_symbol": "UBR3",
  "term_label": "ubiquitin ligase complex",
  "term_id": "GO:0000151",
  "gene": "UniProtKB:Q6ZT12",
  "gene_name": "E3 ubiquitin-protein ligase UBR3"
}